{
  "term_label": "protein sumoylation",
  "gene": "UniProtKB:G2XKQ0",
  "gene_name": "Small ubiquitin-related modifier 5",
  "gene_symbol": "SUMO1P1",
  "term_id": "GO:0016925"
}